{
  "gene_symbol": "PRKCA",
  "gene": "UniProtKB:P17252",
  "term_id": "GO:0004674",
  "gene_name": "Protein kinase C alpha type",
  "term_label": "protein serine/threonine kinase activity"
}